{
  "term_id": "UNKNOWN:0002",
  "term_label": "Unknown biological process",
  "gene_symbol": "CNOT6L",
  "gene": "UniProtKB:Q96LI5",
  "gene_name": "CCR4-NOT transcription complex subunit 6-like"
}